alkylglycerophosphate 2-O-acetyltransferase activity [GO:0047160] (molecular function) Definition: Catalysis of the reaction: 1-alkyl-sn-glycerol 3-phosphate + acetyl-CoA = 1-alkyl-2-acetyl-sn-glycerol 3-phosphate + CoA. Sources: EC:2.3.1.105, RHEA:18557 Also known as: acetyl-CoA:1-alkyl-sn-glycero-3-phosphate 2-O-acetyltransferase activity, alkyllyso-GP:acetyl-CoA acetyltransferase activity Relationships: is a type of O-acetyltransferase activity [GO:0016413]